isopentenyl pyrophosphate transmembrane transporter activity [GO:0170045] (molecular function) Definition: Enables the transfer of isopentenyl pyrophosphate from one side of a membrane to the other. Relationships: is a type of phospholipid transporter activity [GO:0005548]; is a type of organophosphate ester transmembrane transporter activity [GO:0015605]; is a type of lipid transmembrane transporter activity [GO:0170055] Also known as: IPP transmembrane transport activity, isopentenyl diphosphate transmembrane transport activity References: PMID:37813972 Sources: GOC:ew